{
  "term_label": "Unknown molecular function",
  "term_id": "UNKNOWN:0001",
  "gene_symbol": "RUFY2",
  "gene_name": "RUN and FYVE domain-containing protein 2",
  "gene": "UniProtKB:Q8WXA3"
}